{
  "gene_symbol": "SHISA7",
  "term_id": "GO:0050811",
  "gene_name": "Protein shisa-7",
  "term_label": "GABA receptor binding",
  "gene": "UniProtKB:A6NL88"
}